{
  "term_label": "Unknown molecular function",
  "gene": "UniProtKB:A6NGW2",
  "term_id": "UNKNOWN:0001",
  "gene_symbol": "STRCP1",
  "gene_name": "Putative stereocilin-like protein"
}